{
  "gene_name": "Methylated-DNA--protein-cysteine methyltransferase",
  "term_id": "GO:0006281",
  "term_label": "DNA repair",
  "gene": "UniProtKB:P16455",
  "gene_symbol": "MGMT"
}